creatine transmembrane transporter activity [GO:0005308] (molecular function) Definition: Enables the transfer of creatine from one side of a membrane to the other. Creatine is a compound synthesized from the amino acids arginine, glycine, and methionine that occurs in muscle. Relationships: is a type of carboxylic acid transmembrane transporter activity [GO:0046943]; is a type of GO:0072349; is part of GO:0015881 Sources: GOC:ai Subtypes: creatine:sodium symporter activity [GO:0005309]